{
  "gene_name": "ER membrane protein complex subunit 9",
  "gene_symbol": "EMC9",
  "term_label": "EMC complex",
  "gene": "UniProtKB:Q9Y3B6",
  "term_id": "GO:0072546"
}